{
  "gene": "UniProtKB:Q96BD8",
  "gene_symbol": "SKA1",
  "term_label": "chromosome segregation",
  "gene_name": "Spindle and kinetochore-associated protein 1",
  "term_id": "GO:0007059"
}